steroid hormone secretion [GO:0035929] (biological process) Sources: GOC:sl Definition: The regulated release of any steroid that acts as a hormone into the circulatory system. Subtypes: GO:0035930, androgen secretion [GO:0035935], estrogen secretion [GO:0035937], estradiol secretion [GO:0035938], GO:0035943, GO:0042701, ecdysteroid secretion [GO:0045457] Relationships: is a type of endocrine hormone secretion [GO:0060986]; is a type of lipid export from cell [GO:0140353] Regulation: regulated by regulation of steroid hormone secretion [GO:2000831]; negatively regulated by negative regulation of steroid hormone secretion [GO:2000832]; RO_0002213 by GO:2000833